{
  "gene_symbol": "CHST5",
  "gene_name": "Carbohydrate sulfotransferase 5",
  "term_label": "N-acetylglucosamine 6-O-sulfotransferase activity",
  "term_id": "GO:0001517",
  "gene": "UniProtKB:Q9GZS9"
}